{
  "gene_name": "CAAX box protein 1",
  "term_id": "UNKNOWN:0002",
  "gene_symbol": "RTL8C",
  "term_label": "Unknown biological process",
  "gene": "UniProtKB:O15255"
}